{
  "gene_name": "Homeobox protein Hox-C4",
  "gene": "UniProtKB:P09017",
  "term_id": "GO:0009952",
  "gene_symbol": "HOXC4",
  "term_label": "anterior/posterior pattern specification"
}